{
  "gene": "UniProtKB:Q9NUD7",
  "term_id": "UNKNOWN:0001",
  "gene_name": "Uncharacterized protein C20orf96",
  "gene_symbol": "C20orf96",
  "term_label": "Unknown molecular function"
}